regulation of T cell proliferation [GO:0042129] (biological process) Definition: Any process that modulates the frequency, rate or extent of T cell proliferation. Subtypes: GO:0033083, positive regulation of T cell proliferation [GO:0042102], negative regulation of T cell proliferation [GO:0042130], GO:0046006, regulation of T cell homeostatic proliferation [GO:0046013], regulation of alpha-beta T cell proliferation [GO:0046640], regulation of gamma-delta T cell proliferation [GO:0046646] Relationships: is a type of regulation of lymphocyte proliferation [GO:0050670]; is a type of GO:0050863; regulates T cell proliferation [GO:0042098] Sources: GOC:jl Also known as: regulation of T lymphocyte proliferation, regulation of T-cell proliferation, regulation of T-lymphocyte proliferation